{
  "gene": "UniProtKB:P35611",
  "gene_name": "Alpha-adducin",
  "term_id": "GO:0051016",
  "term_label": "barbed-end actin filament capping",
  "gene_symbol": "ADD1"
}